negative regulation of canonical NF-kappaB signal transduction [GO:0043124] (biological process) Relationships: is a type of regulation of canonical NF-kappaB signal transduction [GO:0043122]; is a type of GO:1902532; negatively regulates canonical NF-kappaB signal transduction [GO:0007249] Also known as: down regulation of I-kappaB kinase/NF-kappaB cascade, down-regulation of I-kappaB kinase/NF-kappaB cascade, downregulation of I-kappaB kinase/NF-kappaB cascade, inhibition of I-kappaB kinase/NF-kappaB cascade, negative regulation of I-kappaB kinase/NF-kappaB cascade, negative regulation of I-kappaB kinase/NF-kappaB signaling Sources: GOC:jl Definition: Any process that stops, prevents, or reduces the frequency, rate or extent of a canonical NF-kappaB signaling cascade.